positive regulation of cytoplasmic translational initiation [GO:1904690] (biological process) Relationships: is a type of positive regulation of translational initiation [GO:0045948]; is a type of GO:1904688; RO_0002213 cytoplasmic translational initiation [GO:0002183] Subtypes: GO:1903676, positive regulation of cap-independent translational initiation [GO:1903679] Definition: Any process that activates or increases the frequency, rate or extent of cytoplasmic translational initiation. References: PMID:12242291 Sources: GOC:TermGenie, GO_REF:0000058 Also known as: up regulation of cytoplasmic translational initiation, up-regulation of cytoplasmic translational initiation, upregulation of cytoplasmic translational initiation, activation of cytoplasmic translational initiation